{
  "gene_name": "Myotubularin-related protein 6",
  "gene_symbol": "MTMR6",
  "term_id": "GO:0005737",
  "gene": "UniProtKB:Q9Y217",
  "term_label": "cytoplasm"
}